methyl coenzyme M reductase complex [GO:0044674] (cellular component) References: PMID:9367957 Sources: GOC:mengo_curators Relationships: is a type of transferase complex [GO:1990234] Definition: A hexameric complex consisting of three polypeptides in an alpha2beta2gamma2 arrangement. Involved in the reduction of the coenzyme M-bound methyl group to methane, which is the final step in methanogenesis.